positive regulation of cell proliferation involved in heart valve morphogenesis [GO:0003251] (biological process) Sources: GOC:mtg_heart Definition: Any process that increases the rate, frequency or extent of cell proliferation that contributes to the shaping of a heart valve. Relationships: is a type of GO:0003250; is a type of positive regulation of cell proliferation involved in heart morphogenesis [GO:2000138]; positively regulates cell proliferation involved in heart valve morphogenesis [GO:0003249]